cyclin A1-CDK1 complex [GO:0097121] (cellular component) Relationships: is a type of cyclin-dependent protein kinase holoenzyme complex [GO:0000307] References: PMID:15935619 Sources: GOC:so Definition: A protein complex consisting of cyclin A1 and cyclin-dependent kinase 1 (CDK1). Cyclins are characterized by periodicity in protein abundance throughout the cell cycle. Cyclin-dependent kinases represent a family of serine/threonine protein kinases that become active upon binding to a cyclin regulatory partner.